{
  "term_label": "constitutive heterochromatin formation",
  "term_id": "GO:0140719",
  "gene": "UniProtKB:Q99549",
  "gene_symbol": "MPHOSPH8",
  "gene_name": "M-phase phosphoprotein 8"
}